regulation of myeloid dendritic cell cytokine production [GO:0002733] (biological process) Sources: GOC:add Definition: Any process that modulates the frequency, rate, or extent of myeloid dendritic cell cytokine production. Relationships: is a type of GO:0002730; is_a GO:0002886; regulates myeloid dendritic cell cytokine production [GO:0002372] Subtypes: negative regulation of myeloid dendritic cell cytokine production [GO:0002734], positive regulation of myeloid dendritic cell cytokine production [GO:0002735]